lipopolysaccharide transport system [GO:0062051] (cellular component) Relationships: is a type of transporter complex [GO:1990351] Definition: A protein-containing complex that functions to transport lipopolysaccharide from its site of synthesis at the cytoplasmic membrane across the periplasm to the outer membrane in an ATP-dependent manner. References: PMID:29449493